{
  "term_id": "GO:0007186",
  "gene_symbol": "ADGRG7",
  "term_label": "G protein-coupled receptor signaling pathway",
  "gene_name": "Adhesion G-protein coupled receptor G7",
  "gene": "UniProtKB:Q96K78"
}